{
  "gene_name": "Rab-like protein 2B",
  "gene": "UniProtKB:Q9UNT1",
  "term_id": "GO:0012505",
  "gene_symbol": "RABL2B",
  "term_label": "endomembrane system"
}